{
  "term_label": "Unknown biological process",
  "gene_name": "Myosin light chain 6B",
  "gene_symbol": "MYL6B",
  "gene": "UniProtKB:P14649",
  "term_id": "UNKNOWN:0002"
}